nuclear-transcribed mRNA catabolic process, deadenylation-independent decay [GO:0031086] (biological process) Definition: A pathway of degradation of nuclear-transcribed mRNAs that proceeds through a series of steps that is independent of deadenylation, but requires decapping followed by transcript decay, and that can regulate mRNA stability. Relationships: is a type of nuclear-transcribed mRNA catabolic process [GO:0000956] References: PMID:15225542, PMID:15225544 Sources: GOC:krc Also known as: deadenylation-independent mRNA decay, deadenylylation-independent mRNA decay, mRNA breakdown, deadenylation-independent decay, mRNA catabolic process, deadenylation-independent, mRNA catabolic process, deadenylylation-independent, mRNA catabolism, deadenylation-independent, mRNA catabolism, deadenylation-independent decay, mRNA catabolism, deadenylylation-independent, mRNA degradation, deadenylation-independent decay, nuclear mRNA catabolic process, deadenylation-independent decay